{
  "gene": "UniProtKB:Q58FF8",
  "term_label": "plasma membrane",
  "gene_name": "Putative heat shock protein HSP 90-beta 2",
  "term_id": "GO:0005886",
  "gene_symbol": "HSP90AB2P"
}